{
  "gene_symbol": "DHX58",
  "term_id": "GO:0008270",
  "term_label": "zinc ion binding",
  "gene": "UniProtKB:Q96C10",
  "gene_name": "ATP-dependent RNA helicase DHX58"
}